positive regulation of N-acetylmuramic acid catabolic process [GO:0160159] (biological process) Definition: Any process that activates or increases the frequency, rate or extent of N-acetylmuramic acid catabolic process. Relationships: is a type of positive regulation of catabolic process [GO:0009896]; is a type of GO:0062013; positively regulates N-acetylmuramic acid catabolic process [GO:0097173] References: PMID:18723630